{
  "gene": "UniProtKB:Q8TCU6",
  "gene_symbol": "PREX1",
  "term_id": "GO:0030291",
  "gene_name": "Phosphatidylinositol 3,4,5-trisphosphate-dependent Rac exchanger 1 protein",
  "term_label": "protein serine/threonine kinase inhibitor activity"
}